{
  "gene": "UniProtKB:Q9BYE4",
  "gene_name": "Small proline-rich protein 2G",
  "term_label": "Unknown molecular function",
  "term_id": "UNKNOWN:0001",
  "gene_symbol": "SPRR2G"
}